{
  "gene": "UniProtKB:Q7Z6J8",
  "gene_symbol": "UBE3D",
  "term_label": "nucleus",
  "gene_name": "E3 ubiquitin-protein ligase E3D",
  "term_id": "GO:0005634"
}